{
  "gene_name": "ADP-ribosylation factor 6",
  "term_id": "GO:0001726",
  "gene": "UniProtKB:P62330",
  "term_label": "ruffle",
  "gene_symbol": "ARF6"
}